monounsaturated fatty acid catabolic process [GO:1903965] (biological process) Also known as: monounsaturated fatty acid breakdown, monounsaturated fatty acid catabolism, monounsaturated fatty acid degradation References: PMID:16443825 Sources: GOC:TermGenie, GOC:hjd, GO_REF:0000068 Relationships: is a type of fatty acid catabolic process [GO:0009062]; is a type of monounsaturated fatty acid metabolic process [GO:1903964] Definition: The chemical reactions and pathways resulting in the breakdown of monounsaturated fatty acid.